{
  "gene": "UniProtKB:P01034",
  "gene_symbol": "CST3",
  "gene_name": "Cystatin-C",
  "term_label": "vesicle",
  "term_id": "GO:0031982"
}